{
  "term_id": "GO:0006357",
  "gene_symbol": "ZNF667",
  "term_label": "regulation of transcription by RNA polymerase II",
  "gene_name": "Zinc finger protein 667",
  "gene": "UniProtKB:Q5HYK9"
}